{
  "term_id": "UNKNOWN:0002",
  "gene_symbol": "ECHDC3",
  "gene_name": "Enoyl-CoA hydratase domain-containing protein 3, mitochondrial",
  "term_label": "Unknown biological process",
  "gene": "UniProtKB:Q96DC8"
}